hepatic stellate cell contraction [GO:0061872] (biological process) Regulation: regulated by GO:0061873; positively regulated by positive regulation of hepatic stellate cell contraction [GO:0061874]; negatively regulated by negative regulation of hepatic stellate cell contraction [GO:0061875] References: PMID:24204762 Definition: The actin filament-based process in which cytoplasmic actin filaments slide past one another resulting in contraction of a hepatic stellate cell. Relationships: is a type of actin-mediated cell contraction [GO:0070252]